{
  "gene": "UniProtKB:Q96NW4",
  "gene_name": "Ankyrin repeat domain-containing protein 27",
  "term_id": "GO:0005085",
  "gene_symbol": "ANKRD27",
  "term_label": "guanyl-nucleotide exchange factor activity"
}